alkylhalidase activity [GO:0047651] (molecular function) Definition: Catalysis of the reaction: bromochloromethane + H2O = bromide + chloride + formaldehyde + 2 H+. Also known as: alkyl-halide halidohydrolase activity, haloalkane halidohydrolase activity, halogenase activity Relationships: is a type of GO:0019120 Sources: RHEA:13765